branching involved in mammary gland cord morphogenesis [GO:0060655] (biological process) Regulation: regulated by regulation of branching involved in mammary cord morphogenesis by fat precursor cell-epithelial cell signaling [GO:0060656] Relationships: is a type of GO:0060444; is part of mammary gland cord morphogenesis [GO:0060652] Definition: The process in which the branching structure of the mammary gland cord is generated and organized. The mammary gland cord is a solid epithelial structure that will hollow out, forming the mammary duct. References: PMID:12558599 Sources: GOC:dph